{
  "term_id": "GO:1990756",
  "gene": "UniProtKB:Q5VTA0",
  "gene_name": "PRAME family member 17",
  "gene_symbol": "PRAMEF17",
  "term_label": "ubiquitin-like ligase-substrate adaptor activity"
}